epicardium-derived cardiac fibroblast cell differentiation [GO:0060938] (biological process) Sources: GOC:mtg_heart Definition: The process in which an epicardial cell acquires the specialized structural and/or functional features of a cardiac fibroblast. A cardiac fibroblast is a connective tissue cell in the heart which secretes an extracellular matrix rich in collagen and other macromolecules. Relationships: is a type of cardiac fibroblast cell differentiation [GO:0060935]